negative regulation of appetite [GO:0032099] (BP) Relationships: is a type of negative regulation of response to food [GO:0032096]; is a type of regulation of appetite [GO:0032098] Also known as: down regulation of appetite, down-regulation of appetite, downregulation of appetite, inhibition of appetite, appetite suppression, negative regulation of hunger Definition: Any process that reduces appetite. Sources: GOC:add Subtypes: negative regulation of appetite by leptin-mediated signaling pathway [GO:0038108]